{
  "term_id": "UNKNOWN:0002",
  "gene": "UniProtKB:Q8IWE2",
  "term_label": "Unknown biological process",
  "gene_symbol": "FAM114A1",
  "gene_name": "Protein NOXP20"
}